{
  "term_label": "cytoplasmic side of lysosomal membrane",
  "term_id": "GO:0098574",
  "gene_symbol": "BORCS5",
  "gene_name": "BLOC-1-related complex subunit 5",
  "gene": "UniProtKB:Q969J3"
}